{
  "gene": "UniProtKB:Q9BRD0",
  "term_id": "GO:0005684",
  "gene_symbol": "BUD13",
  "term_label": "U2-type spliceosomal complex",
  "gene_name": "BUD13 homolog"
}